{
  "gene": "UniProtKB:Q8WXG1",
  "gene_name": "S-adenosylmethionine-dependent nucleotide dehydratase RSAD2",
  "term_label": "positive regulation of immune response",
  "term_id": "GO:0050778",
  "gene_symbol": "RSAD2"
}